{
  "gene_name": "Histone H2A type 1",
  "term_label": "nucleus",
  "term_id": "GO:0005634",
  "gene": "UniProtKB:P0C0S8",
  "gene_symbol": "H2AC17"
}